{
  "gene_symbol": "TMEM183A",
  "term_id": "GO:0019005",
  "gene_name": "Transmembrane protein 183A",
  "gene": "UniProtKB:Q8IXX5",
  "term_label": "SCF ubiquitin ligase complex"
}